{
  "gene_symbol": "RAB5A",
  "term_label": "intracellular protein transport",
  "term_id": "GO:0006886",
  "gene_name": "Ras-related protein Rab-5A",
  "gene": "UniProtKB:P20339"
}